pyruvate family amino acid biosynthetic process [GO:0009079] (biological process) Relationships: is a type of L-amino acid biosynthetic process [GO:0170034]; is a type of GO:0170038 Subtypes: L-leucine biosynthetic process [GO:0009098], L-valine biosynthetic process [GO:0009099], L-alanine biosynthetic process [GO:0042852] Sources: GOC:jl Also known as: pyruvate family amino acid anabolism, pyruvate family amino acid biosynthesis, pyruvate family amino acid formation, pyruvate family amino acid synthesis Definition: The chemical reactions and pathways resulting in the formation of any amino acid that requires pyruvate for its synthesis, e.g. alanine.